regulation of adherens junction organization [GO:1903391] (biological process) Definition: Any process that modulates the frequency, rate or extent of adherens junction organization. Relationships: is a type of regulation of cellular component organization [GO:0051128]; regulates GO:0034332 References: PMID:21724833 Sources: GOC:TermGenie, GOC:als, GO_REF:0000058 Also known as: regulation of adherens junction assembly and maintenance, regulation of adherens junction organisation Subtypes: negative regulation of adherens junction organization [GO:1903392], positive regulation of adherens junction organization [GO:1903393]